{
  "gene_name": "Leucine-rich repeat-containing protein 37A",
  "term_id": "UNKNOWN:0002",
  "gene": "UniProtKB:A6NMS7",
  "term_label": "Unknown biological process",
  "gene_symbol": "LRRC37A"
}